{
  "term_label": "plasma membrane",
  "gene": "UniProtKB:P30556",
  "gene_symbol": "AGTR1",
  "gene_name": "Type-1 angiotensin II receptor",
  "term_id": "GO:0005886"
}